{
  "gene_name": "Olfactory receptor 8J2",
  "gene_symbol": "OR8J2",
  "term_label": "Unknown molecular function",
  "term_id": "UNKNOWN:0001",
  "gene": "UniProtKB:Q8NGG1"
}